1,2,4-trichlorobenzene catabolic process [GO:0018911] (biological process) Relationships: is a type of GO:0009056; is a type of GO:0042537; is a type of organohalogen metabolic process [GO:0090345] Definition: The chemical reactions and pathways resulting in the breakdown of 1,2,4-trichlorobenzene, a derivative of benzene with chlorine atoms attached to positions 1, 2 and 4 of the ring. It is a colorless liquid used as a solvent in chemical manufacturing, in dyes and intermediates, dielectric fluid, synthetic transformer oils, lubricants, heat-transfer medium and insecticides. References: PMID:1987135 Also known as: 1,2,4-trichlorobenzene metabolic process, 1,2,4-trichlorobenzene metabolism